{
  "gene": "UniProtKB:Q9BS34",
  "gene_name": "Zinc finger protein 670",
  "term_label": "RNA polymerase II cis-regulatory region sequence-specific DNA binding",
  "term_id": "GO:0000978",
  "gene_symbol": "ZNF670"
}